{
  "term_id": "GO:0030010",
  "gene_symbol": "PARD3",
  "gene": "UniProtKB:Q8TEW0",
  "term_label": "establishment of cell polarity",
  "gene_name": "Partitioning defective 3 homolog"
}